N-acetylglucosamine transport [GO:0015764] (biological process) Sources: GOC:mah Definition: The directed movement of N-acetylglucosamine into, out of or within a cell, or between cells, by means of some agent such as a transporter or pore. Relationships: is a type of carbohydrate derivative transport [GO:1901264]